{
  "gene": "UniProtKB:Q86X67",
  "gene_symbol": "NUDT13",
  "term_label": "Unknown biological process",
  "term_id": "UNKNOWN:0002",
  "gene_name": "NAD(P)H pyrophosphatase NUDT13, mitochondrial"
}